{
  "gene": "UniProtKB:Q9ULD9",
  "term_label": "nucleus",
  "gene_symbol": "ZNF608",
  "term_id": "GO:0005634",
  "gene_name": "Zinc finger protein 608"
}